{
  "gene": "UniProtKB:Q15700",
  "gene_name": "Disks large homolog 2",
  "term_label": "nervous system development",
  "term_id": "GO:0007399",
  "gene_symbol": "DLG2"
}